regulation of antimicrobial peptide production [GO:0002784] (biological process) Sources: GOC:add Definition: Any process that modulates the frequency, rate, or extent of antimicrobial peptide production. Subtypes: positive regulation of antimicrobial peptide production [GO:0002225], negative regulation of antimicrobial peptide production [GO:0002785], regulation of antibacterial peptide production [GO:0002786], regulation of antifungal peptide production [GO:0002788], regulation of antimicrobial peptide secretion [GO:0002794], GO:0002805 Relationships: is_a regulation of production of molecular mediator of immune response [GO:0002700]; is a type of regulation of antimicrobial humoral response [GO:0002759]; regulates antimicrobial peptide production [GO:0002775]